{
  "gene_symbol": "IFITM3",
  "term_label": "defense response to virus",
  "gene_name": "Interferon-induced transmembrane protein 3",
  "term_id": "GO:0051607",
  "gene": "UniProtKB:Q01628"
}